GPI anchored protein biosynthesis [GO:0180046] (biological process) Definition: Any process leading to the post-translational modification of a protein with a GPI anchor to achieve full functional capacity of the protein. Sources: GOC:vw Relationships: is a type of protein maturation [GO:0051604]